{
  "gene": "UniProtKB:A0A3B3IU46",
  "gene_symbol": "RAMACL",
  "term_id": "GO:0008047",
  "gene_name": "RNA guanine-N7 methyltransferase-activating subunit-like protein",
  "term_label": "enzyme activator activity"
}